{
  "gene_symbol": "CLEC4M",
  "gene_name": "C-type lectin domain family 4 member M",
  "gene": "UniProtKB:Q9H2X3",
  "term_label": "pattern recognition receptor activity",
  "term_id": "GO:0038187"
}